{
  "term_id": "GO:0005615",
  "gene": "UniProtKB:P13497",
  "gene_name": "Bone morphogenetic protein 1",
  "term_label": "extracellular space",
  "gene_symbol": "BMP1"
}